{
  "term_label": "ubiquitin-like ligase-substrate adaptor activity",
  "term_id": "GO:1990756",
  "gene_name": "Putative PRAME family member 13",
  "gene_symbol": "PRAMEF13",
  "gene": "UniProtKB:Q5VWM6"
}